{
  "gene_name": "Zeta-sarcoglycan",
  "term_id": "GO:0048738",
  "gene": "UniProtKB:Q96LD1",
  "gene_symbol": "SGCZ",
  "term_label": "cardiac muscle tissue development"
}